{
  "term_label": "postsynaptic density membrane",
  "gene_symbol": "GRM1",
  "term_id": "GO:0098839",
  "gene": "UniProtKB:Q13255",
  "gene_name": "Metabotropic glutamate receptor 1"
}